{
  "gene_name": "Mitochondrial fission process protein 1",
  "term_label": "mitochondrial fission",
  "gene": "UniProtKB:Q9UDX5",
  "gene_symbol": "MTFP1",
  "term_id": "GO:0000266"
}